{
  "gene": "UniProtKB:Q9BSH4",
  "term_label": "Unknown molecular function",
  "gene_name": "Translational activator of cytochrome c oxidase 1",
  "gene_symbol": "TACO1",
  "term_id": "UNKNOWN:0001"
}